cranial skeletal system development [GO:1904888] (biological process) Definition: The process whose specific outcome is the progression of a cranial skeletal system over time, from its formation to the mature structure. The cranial skeletal system is the skeletal subdivision of the head, and includes the skull (cranium plus mandible), pharyngeal and/or hyoid apparatus. References: PMID:11262227 Sources: GOC:PARL, GOC:TermGenie, GOC:bf, GO_REF:0000094 Also known as: cranial skeleton development, craniofacial development, osteocranium development, cranium development Relationships: is a type of anatomical structure development [GO:0048856]